{
  "gene": "UniProtKB:O14867",
  "term_id": "UNKNOWN:0003",
  "gene_name": "Transcription regulator protein BACH1",
  "gene_symbol": "BACH1",
  "term_label": "Unknown cellular component"
}